{
  "gene_name": "SH3-containing GRB2-like protein 3-interacting protein 1",
  "gene": "UniProtKB:Q9BQI5",
  "gene_symbol": "SGIP1",
  "term_label": "Unknown biological process",
  "term_id": "UNKNOWN:0002"
}